{
  "term_label": "neuron projection development",
  "term_id": "GO:0031175",
  "gene_symbol": "RAPGEF2",
  "gene": "UniProtKB:Q9Y4G8",
  "gene_name": "Rap guanine nucleotide exchange factor 2"
}